negative regulation of myofibroblast cell apoptotic process [GO:1904521] (biological process) Definition: Any process that stops, prevents or reduces the frequency, rate or extent of myofibroblast cell apoptotic process. References: PMID:26119034 Sources: GOC:TermGenie, GO_REF:0000058 Also known as: down regulation of MFB apoptotic process, down regulation of myofibroblast cell apoptotic process, down-regulation of MFB apoptotic process, down-regulation of myofibroblast cell apoptotic process, downregulation of MFB apoptotic process, downregulation of myofibroblast cell apoptotic process, negative regulation of MFB apoptotic process, down regulation of MFB apoptosis, down regulation of myofibroblast cell apoptosis, down-regulation of MFB apoptosis, down-regulation of myofibroblast cell apoptosis, downregulation of MFB apoptosis, downregulation of myofibroblast cell apoptosis, inhibition of MFB apoptosis, inhibition of MFB apoptotic process, inhibition of myofibroblast cell apoptosis, inhibition of myofibroblast cell apoptotic process, negative regulation of MFB apoptosis, negative regulation of myofibroblast cell apoptosis Relationships: is a type of GO:0043066; is a type of regulation of myofibroblast cell apoptotic process [GO:1904520]; negatively regulates myofibroblast cell apoptotic process [GO:1904516]